RNA localization [GO:0006403] (biological process) Definition: A process in which RNA is transported to, or maintained in, a specific location. Relationships: is a type of macromolecule localization [GO:0033036] Subtypes: GO:0007316, GO:0008298, mitochondrial RNA localization [GO:0019093], snoRNA localization [GO:0048254], GO:0090672, RNA localization to nucleus [GO:0090685], RNA localization to chromatin [GO:1990280] Sources: GOC:ai Also known as: RNA localisation, establishment and maintenance of RNA localization